{
  "term_label": "endoplasmic reticulum membrane",
  "gene_symbol": "MARCHF6",
  "gene": "UniProtKB:O60337",
  "gene_name": "E3 ubiquitin-protein ligase MARCHF6",
  "term_id": "GO:0005789"
}